light-dependent bacteriochlorophyll biosynthetic process [GO:0036069] (biological process) Also known as: light dependent bacteriochlorophyll biosynthetic process, light-dependent bacteriochlorophyll anabolism, light-dependent bacteriochlorophyll biosynthesis, light-dependent bacteriochlorophyll formation, light-dependent bacteriochlorophyll synthesis Relationships: is a type of bacteriochlorophyll biosynthetic process [GO:0030494]; is a type of GO:0036067 Definition: The chemical reactions and pathways resulting in the formation of a bacteriochlorophyll, which occur in the presence of light. Bacteriochlorophylls are any of the chlorophylls of photosynthetic bacteria; they differ structurally from the chlorophylls of higher plants. References: PMID:12242396 Sources: GOC:yaf